{
  "term_id": "GO:0005794",
  "gene_name": "Beta-galactoside alpha-2,6-sialyltransferase 2",
  "term_label": "Golgi apparatus",
  "gene_symbol": "ST6GAL2",
  "gene": "UniProtKB:Q96JF0"
}